muscle cell projection [GO:0036194] (cellular component) Definition: A prolongation or process extending from a muscle cell. A muscle cell is a mature contractile cell, commonly known as a myocyte. This cell has as part of its cytoplasm myofibrils organized in various patterns. References: PMID:15930100, PMID:22464329 Sources: CL:0000187, GOC:kmv Relationships: is_a plasma membrane bounded cell projection [GO:0120025] Also known as: myocyte projection, muscle arm, myopodia